norepinephrine-epinephrine-mediated vasodilation involved in regulation of systemic arterial blood pressure [GO:0002025] (biological process) References: PMID:10358008 Sources: GOC:mtg_cardio Also known as: noradrenaline-adrenaline vasodilation involved in regulation of blood pressure, norepinephrine-epinephrine vasodilation during blood pressure regulation, vasodilation by norepinephrine-epinephrine involved in regulation of systemic arterial blood pressure Relationships: is_a negative regulation of systemic arterial blood pressure [GO:0003085]; is a type of vasodilation [GO:0042311]; BFO_0000050 regulation of systemic arterial blood pressure by norepinephrine-epinephrine [GO:0001993] Definition: A process that results in an increase in the diameter of an artery during the norepinephrine-epinephrine response to blood pressure change.